{
  "gene": "UniProtKB:Q6P1M9",
  "term_label": "Unknown biological process",
  "gene_symbol": "ARMCX5",
  "gene_name": "Armadillo repeat-containing X-linked protein 5",
  "term_id": "UNKNOWN:0002"
}